{
  "gene_symbol": "KIAA1549",
  "term_label": "Unknown biological process",
  "gene": "UniProtKB:Q9HCM3",
  "term_id": "UNKNOWN:0002",
  "gene_name": "UPF0606 protein KIAA1549"
}